metaphase/anaphase transition of meiosis I [GO:1990949] (BP) Definition: The cell cycle process in which a cell progresses from metaphase to anaphase as part of meiosis I. Also known as: meiosis I metaphase/anaphase transition, first meiotic metaphase/anaphase transition Relationships: is a type of metaphase/anaphase transition of meiotic cell cycle [GO:0044785]; is a type of meiosis I cell cycle process [GO:0061982] Regulation: regulated by GO:1905186; negatively regulated by negative regulation of metaphase/anaphase transition of meiosis I [GO:1905187]; positively regulated by positive regulation of metaphase/anaphase transition of meiosis I [GO:1905188] Sources: ISBN:0815316194